{
  "term_label": "mitochondrial small ribosomal subunit",
  "term_id": "GO:0005763",
  "gene": "UniProtKB:Q9BYN8",
  "gene_name": "Small ribosomal subunit protein mS26",
  "gene_symbol": "MRPS26"
}